{
  "gene": "UniProtKB:Q9H3R1",
  "term_id": "GO:0019213",
  "gene_name": "Bifunctional heparan sulfate N-deacetylase_N-sulfotransferase 4",
  "gene_symbol": "NDST4",
  "term_label": "deacetylase activity"
}